{
  "term_id": "GO:1902723",
  "gene_symbol": "AKIRIN1",
  "gene": "UniProtKB:Q9H9L7",
  "gene_name": "Akirin-1",
  "term_label": "negative regulation of skeletal muscle satellite cell proliferation"
}